{
  "gene": "UniProtKB:Q9UDV7",
  "term_id": "GO:0000978",
  "gene_symbol": "ZNF282",
  "term_label": "RNA polymerase II cis-regulatory region sequence-specific DNA binding",
  "gene_name": "Zinc finger protein 282"
}